regulation of mast cell apoptotic process [GO:0033025] (biological process) Relationships: is a type of GO:0002682; is a type of regulation of myeloid cell apoptotic process [GO:0033032]; is a type of regulation of leukocyte apoptotic process [GO:2000106]; regulates mast cell apoptotic process [GO:0033024] Also known as: regulation of mast cell apoptosis Definition: Any process that modulates the frequency, rate, or extent of mast cell apoptotic process. Sources: GOC:add, GOC:mtg_apoptosis Subtypes: negative regulation of mast cell apoptotic process [GO:0033026], positive regulation of mast cell apoptotic process [GO:0033027]